{
  "gene_symbol": "WSCD1",
  "gene": "UniProtKB:Q658N2",
  "gene_name": "Sialate:O-sulfotransferase 1",
  "term_label": "Unknown cellular component",
  "term_id": "UNKNOWN:0003"
}